regulation of postsynaptic cytosolic calcium ion concentration [GO:0099566] (BP) Sources: GOC:dos Also known as: regulation of postsynaptic cytosolic calcium levels Definition: Any process that regulates the concentration of calcium in the postsynaptic cytosol. Relationships: is a type of GO:0051480; occurs in GO:0098794